muscle contraction [GO:0006936] (biological process) Definition: A process in which force is generated within muscle tissue, resulting in a change in muscle geometry. Force generation involves a chemo-mechanical energy conversion step that is carried out by the actin/myosin complex activity, which generates force through ATP hydrolysis. Relationships: is a type of GO:0003012 Sources: GOC:ef, GOC:mtg_muscle, ISBN:0198506732 Subtypes: smooth muscle contraction [GO:0006939], striated muscle contraction [GO:0006941] Regulation: regulated by GO:0006937; negatively regulated by negative regulation of muscle contraction [GO:0045932]; positively regulated by positive regulation of muscle contraction [GO:0045933]